{
  "term_id": "GO:0008247",
  "gene": "UniProtKB:Q15102",
  "gene_name": "Platelet-activating factor acetylhydrolase IB subunit alpha1",
  "gene_symbol": "PAFAH1B3",
  "term_label": "1-alkyl-2-acetylglycerophosphocholine esterase complex"
}